{
  "gene": "UniProtKB:Q13398",
  "term_id": "GO:0000978",
  "term_label": "RNA polymerase II cis-regulatory region sequence-specific DNA binding",
  "gene_name": "Zinc finger protein 211",
  "gene_symbol": "ZNF211"
}